{
  "gene_name": "UV-stimulated scaffold protein A",
  "gene_symbol": "UVSSA",
  "gene": "UniProtKB:Q2YD98",
  "term_id": "GO:0005694",
  "term_label": "chromosome"
}